{
  "gene_symbol": "KIF2C",
  "term_id": "GO:0007018",
  "term_label": "microtubule-based movement",
  "gene_name": "Kinesin-like protein KIF2C",
  "gene": "UniProtKB:Q99661"
}